{
  "gene": "UniProtKB:Q15047",
  "term_id": "GO:0010629",
  "gene_symbol": "SETDB1",
  "gene_name": "Histone-lysine N-methyltransferase SETDB1",
  "term_label": "negative regulation of gene expression"
}